{
  "gene": "UniProtKB:A1A5D9",
  "term_label": "vesicle transport along microtubule",
  "gene_name": "BICD family-like cargo adapter 2",
  "gene_symbol": "BICDL2",
  "term_id": "GO:0047496"
}